{
  "gene_name": "Tetraspanin-4",
  "gene_symbol": "TSPAN4",
  "gene": "UniProtKB:O14817",
  "term_label": "Unknown biological process",
  "term_id": "UNKNOWN:0002"
}